pimeloyl-CoA dehydrogenase activity [GO:0018515] (molecular function) Relationships: is a type of oxidoreductase activity, acting on the CH-CH group of donors, NAD or NADP as acceptor [GO:0016628] Also known as: pimeloyl-CoA:NAD+ oxidoreductase activity Sources: EC:1.3.1.62, RHEA:19665 Definition: Catalysis of the reaction: NAD+ + pimelyl-CoA = 2,3-didehydropimeloyl-CoA + H+ + NADH.